{
  "term_id": "GO:0005634",
  "term_label": "nucleus",
  "gene": "UniProtKB:Q5VYK3",
  "gene_symbol": "ECPAS",
  "gene_name": "Proteasome adapter and scaffold protein ECM29"
}